{
  "gene": "UniProtKB:Q8IWJ2",
  "gene_symbol": "GCC2",
  "term_id": "UNKNOWN:0001",
  "gene_name": "GRIP and coiled-coil domain-containing protein 2",
  "term_label": "Unknown molecular function"
}